sulfur amino acid catabolic process [GO:0000098] (biological process) Also known as: sulfur amino acid breakdown, sulfur amino acid catabolism, sulfur amino acid degradation, sulphur amino acid catabolic process, sulphur amino acid catabolism Subtypes: GO:0009087, GO:0009093, homocysteine catabolic process [GO:0043418], ergothioneine catabolic process [GO:0052700] Sources: GOC:ai Definition: The chemical reactions and pathways resulting in the breakdown of amino acids containing sulfur, comprising cysteine, methionine and selenocysteine. Relationships: is a type of sulfur amino acid metabolic process [GO:0000096]; is a type of sulfur compound catabolic process [GO:0044273]; is a type of carboxylic acid catabolic process [GO:0046395]